{
  "gene_name": "Beta-defensin 121",
  "term_label": "Unknown cellular component",
  "gene": "UniProtKB:Q5J5C9",
  "term_id": "UNKNOWN:0003",
  "gene_symbol": "DEFB121"
}